response to retinoic acid [GO:0032526] (biological process) Subtypes: GO:0071300 Sources: GOC:sl Also known as: response to vitamin A acid Definition: Any process that results in a change in state or activity of a cell or an organism (in terms of movement, secretion, enzyme production, gene expression, etc.) as a result of a retinoic acid stimulus. Relationships: is a type of GO:0033993; is a type of response to oxygen-containing compound [GO:1901700]